{
  "gene_symbol": "SLC27A5",
  "term_id": "GO:0005324",
  "gene": "UniProtKB:Q9Y2P5",
  "term_label": "long-chain fatty acid transmembrane transporter activity",
  "gene_name": "Long-chain fatty acid transport protein 5"
}